{
  "term_id": "GO:0001726",
  "gene_symbol": "FSCN1",
  "gene_name": "Fascin",
  "gene": "UniProtKB:Q16658",
  "term_label": "ruffle"
}